{
  "gene": "UniProtKB:Q9BWF3",
  "term_label": "mRNA binding",
  "gene_symbol": "RBM4",
  "gene_name": "RNA-binding protein 4",
  "term_id": "GO:0003729"
}